{
  "gene_symbol": "TCF19",
  "term_id": "GO:0010468",
  "term_label": "regulation of gene expression",
  "gene_name": "Transcription factor 19",
  "gene": "UniProtKB:Q9Y242"
}